{
  "gene_symbol": "COL4A2",
  "term_label": "collagen-activated tyrosine kinase receptor signaling pathway",
  "gene": "UniProtKB:P08572",
  "term_id": "GO:0038063",
  "gene_name": "Collagen alpha-2(IV) chain"
}